regulation of glucocorticoid biosynthetic process [GO:0031946] (biological process) Relationships: is a type of GO:0031943; is a type of regulation of steroid hormone biosynthetic process [GO:0090030]; regulates GO:0006704 Definition: Any process that modulates the frequency, rate or extent of the chemical reactions and pathways resulting in the formation of glucocorticoids. Sources: GOC:mah Subtypes: negative regulation of glucocorticoid biosynthetic process [GO:0031947], positive regulation of glucocorticoid biosynthetic process [GO:0031948], regulation of cortisol biosynthetic process [GO:2000064]